{
  "gene_symbol": "CRYBB2",
  "gene_name": "Beta-crystallin B2",
  "term_id": "GO:0007601",
  "gene": "UniProtKB:P43320",
  "term_label": "visual perception"
}